{
  "gene_symbol": "ICE2",
  "gene": "UniProtKB:Q659A1",
  "term_id": "GO:0042795",
  "gene_name": "Little elongation complex subunit 2",
  "term_label": "snRNA transcription by RNA polymerase II"
}